lipoprotein lipase activity [GO:0004465] (molecular function) Sources: EC:3.1.1.34, GOC:bf Regulation: negatively regulated by negative regulation of lipoprotein lipase activity [GO:0051005]; RO_0002213 by positive regulation of lipoprotein lipase activity [GO:0051006]; positively regulated by lipoprotein lipase activator activity [GO:0060230] Relationships: is_a GO:0004806 Definition: Catalysis of the reaction: triacylglycerol + H2O = diacylglycerol + a carboxylate, where the triacylglycerol is part of a lipoprotein. May also hydrolyze diacylglycerol and phospholipids present in lipoproteins. Also known as: clearing factor lipase activity, diacylglycerol hydrolase activity, diacylglycerol lipase activity, diglyceride lipase activity, lipemia-clearing factor, postheparin esterase activity, postheparin lipase activity, triacylglycero-protein acylhydrolase activity